{
  "term_id": "GO:0051723",
  "gene_symbol": "PPME1",
  "gene": "UniProtKB:Q9Y570",
  "gene_name": "Protein phosphatase methylesterase 1",
  "term_label": "protein methylesterase activity"
}